regulation of odontogenesis of dentin-containing tooth [GO:0042487] (biological process) Subtypes: GO:0042488, GO:0042489 Relationships: is a type of GO:0042481; regulates odontogenesis of dentin-containing tooth [GO:0042475] Definition: Any process that modulates the frequency, rate or extent of the formation and development of teeth, the hard, bony appendages which are borne on the jaws, or on other bones in the walls of the mouth or pharynx of most vertebrates. References: PMID:15355794 Sources: GOC:jl, GOC:mtg_sensu Also known as: regulation of odontogenesis of dentine-containing teeth, regulation of odontogenesis of dentine-containing tooth